{
  "term_id": "UNKNOWN:0003",
  "term_label": "Unknown cellular component",
  "gene_symbol": "NPIPA5",
  "gene": "UniProtKB:E9PKD4",
  "gene_name": "Nuclear pore complex-interacting protein family member A5"
}